{
  "term_id": "GO:0016567",
  "gene_name": "Ankyrin repeat and SOCS box protein 11",
  "gene_symbol": "ASB11",
  "gene": "UniProtKB:Q8WXH4",
  "term_label": "protein ubiquitination"
}